{
  "term_id": "GO:0031386",
  "term_label": "protein tag activity",
  "gene_name": "Ubiquitin-related modifier 1",
  "gene": "UniProtKB:Q9BTM9",
  "gene_symbol": "URM1"
}